L-methionine N-acyltransferase activity [GO:0103045] (molecular function) Relationships: is a type of L-amino-acid N-acetyltransferase activity [GO:0140085] Sources: RHEA:44144 Definition: Catalysis of the reaction: L-methionine + acetyl-CoA = N-acetyl-L-methionine + coenzyme A + H+.